{
  "gene": "UniProtKB:Q63HK3",
  "term_label": "RNA polymerase II cis-regulatory region sequence-specific DNA binding",
  "gene_name": "Zinc finger protein with KRAB and SCAN domains 2",
  "term_id": "GO:0000978",
  "gene_symbol": "ZKSCAN2"
}